{
  "gene_symbol": "PGM5",
  "term_id": "GO:0030239",
  "gene_name": "Phosphoglucomutase-like protein 5",
  "term_label": "myofibril assembly",
  "gene": "UniProtKB:Q15124"
}